{
  "term_label": "Unknown molecular function",
  "gene_symbol": "AADACL2",
  "term_id": "UNKNOWN:0001",
  "gene_name": "Arylacetamide deacetylase-like 2",
  "gene": "UniProtKB:Q6P093"
}